{
  "term_label": "receptor complex",
  "term_id": "GO:0043235",
  "gene_symbol": "AMHR2",
  "gene_name": "Anti-Muellerian hormone type-2 receptor",
  "gene": "UniProtKB:Q16671"
}